{
  "term_id": "GO:0016192",
  "term_label": "vesicle-mediated transport",
  "gene": "UniProtKB:Q8NC96",
  "gene_name": "Adaptin ear-binding coat-associated protein 1",
  "gene_symbol": "NECAP1"
}